{
  "term_id": "GO:0005096",
  "term_label": "GTPase activator activity",
  "gene": "UniProtKB:Q86UD7",
  "gene_name": "TBC1 domain family member 26",
  "gene_symbol": "TBC1D26"
}